{
  "gene": "UniProtKB:Q96H35",
  "gene_name": "Probable RNA-binding protein 18",
  "term_label": "Unknown biological process",
  "gene_symbol": "RBM18",
  "term_id": "UNKNOWN:0002"
}